regulation of actin filament annealing [GO:0110054] (biological process) Definition: Any process that modulates the frequency, rate or extent of actin filament annealing, i.e. the end-to-end joining of existing actin filaments. Subtypes: negative regulation of actin filament annealing [GO:0110055], positive regulation of actin filament annealing [GO:0110056] References: PMID:10585915, PMID:11575927, PMID:15743909, PMID:19244341 Sources: GOC:mah Relationships: is a type of GO:0110053